miRNA export from nucleus [GO:0061716] (biological process) References: PMID:15738428, PMID:21554756 Sources: GOC:BHF, GOC:BHF_miRNA, GOC:rph Relationships: is_a RNA export from nucleus [GO:0006405]; is a type of miRNA transport [GO:1990428] Definition: The directed movement of a processed miRNA from the nucleus to the cytoplasm.